{
  "gene_name": "Spatacsin",
  "term_id": "GO:0030424",
  "gene": "UniProtKB:Q96JI7",
  "term_label": "axon",
  "gene_symbol": "SPG11"
}